lymphatic vascular process in circulatory system [GO:1990183] (biological process) Relationships: is a type of vascular process in circulatory system [GO:0003018] Subtypes: regulation of lymphatic vascular permeability [GO:1990185], regulation of lymphatic vessel size [GO:1990186] References: PMID:21576390 Definition: A circulatory process that occurs at the level of the lymphatic vasculature.